{
  "gene_symbol": "RAD21L1",
  "term_label": "replication-born double-strand break repair via sister chromatid exchange",
  "gene": "UniProtKB:Q9H4I0",
  "term_id": "GO:1990414",
  "gene_name": "Double-strand-break repair protein rad21-like protein 1"
}